{
  "term_label": "endoplasmic reticulum",
  "gene_symbol": "LCLAT1",
  "term_id": "GO:0005783",
  "gene_name": "Lysocardiolipin acyltransferase 1",
  "gene": "UniProtKB:Q6UWP7"
}